{
  "term_id": "UNKNOWN:0002",
  "gene_name": "Putative uncharacterized protein C5orf58",
  "gene_symbol": "C5orf58",
  "term_label": "Unknown biological process",
  "gene": "UniProtKB:C9J3I9"
}